{
  "term_id": "GO:1902711",
  "gene": "UniProtKB:P28476",
  "gene_name": "Gamma-aminobutyric acid receptor subunit rho-2",
  "gene_symbol": "GABRR2",
  "term_label": "GABA-A receptor complex"
}